positive regulation of DNA metabolic process [GO:0051054] (BP) Definition: Any process that activates or increases the frequency, rate or extent of the chemical reactions and pathways involving DNA. Sources: GOC:ai Also known as: positive regulation of DNA metabolism, up regulation of DNA metabolic process, up-regulation of DNA metabolic process, upregulation of DNA metabolic process, activation of DNA metabolic process, stimulation of DNA metabolic process Relationships: is a type of positive regulation of macromolecule metabolic process [GO:0010604]; is a type of GO:0051052; positively regulates DNA metabolic process [GO:0006259] Subtypes: positive regulation of deoxyribonuclease activity [GO:0032077], positive regulation of telomere maintenance [GO:0032206], positive regulation of DNA repair [GO:0045739], positive regulation of DNA replication [GO:0045740], GO:0045911, GO:0060383, positive regulation of strand invasion [GO:0098530], positive regulation of DNA strand resection involved in replication fork processing [GO:0106253], positive regulation of mitotic recombination-dependent replication fork processing [GO:0120292], GO:0141170, positive regulation of mitochondrial DNA metabolic process [GO:1901860], positive regulation of meiotic DNA double-strand break formation [GO:1903343], GO:1903626, positive regulation of DNA biosynthetic process [GO:2000573]